female meiosis chromosome separation [GO:0051309] (biological process) Definition: The process in which paired chromosomes are physically detached from each other during female meiosis. Sources: GOC:ai Relationships: is a type of female meiosis chromosome segregation [GO:0016321]; is a type of meiotic chromosome separation [GO:0051307] Also known as: chromosome separation during female meiosis, female meiosis chromosome resolution